{
  "gene": "UniProtKB:P41250",
  "gene_symbol": "GARS1",
  "term_id": "GO:0005737",
  "term_label": "cytoplasm",
  "gene_name": "Glycine--tRNA ligase"
}